{
  "term_label": "Unknown molecular function",
  "gene_name": "Keratin-associated protein 2-1",
  "gene_symbol": "KRTAP2-1",
  "term_id": "UNKNOWN:0001",
  "gene": "UniProtKB:Q9BYU5"
}